single-stranded DNA 5'-3' DNA exonuclease activity [GO:0045145] (molecular function) Also known as: single-stranded DNA specific 5'-3' exodeoxyribonuclease activity, ssDNA-specific 5'-3' exodeoxyribonuclease activity References: PMID:20086101 Sources: GOC:ai, GOC:elh Relationships: is a type of single-stranded DNA exodeoxyribonuclease activity [GO:0008297]; is a type of 5'-3' DNA exonuclease activity [GO:0035312] Definition: Catalysis of the sequential cleavage of nucleotides (such as mononucleotides or dinucleotides) from a free 5' terminus of a single-stranded DNA molecule.